{
  "gene_name": "Uroplakin-3b",
  "term_label": "Unknown molecular function",
  "gene_symbol": "UPK3B",
  "gene": "UniProtKB:Q9BT76",
  "term_id": "UNKNOWN:0001"
}